{
  "gene_name": "Protein EFR3 homolog A",
  "gene": "UniProtKB:Q14156",
  "gene_symbol": "EFR3A",
  "term_label": "Unknown molecular function",
  "term_id": "UNKNOWN:0001"
}